protein-containing complex localization [GO:0031503] (biological process) Subtypes: protein-DNA complex transport [GO:0015869], GO:0031144, gamma-tubulin complex localization [GO:0033566], RITS complex localization [GO:0034630], GO:0035853, GO:0044382, exocyst localization [GO:0051601], GO:0051664, P-TEFb-cap methyltransferase complex localization [GO:0070817], chromosome passenger complex localization to kinetochore [GO:0072356], SHREC complex localization [GO:0072688], SAGA complex localization to transcription regulatory region [GO:0072742], centromere localization [GO:0072765], GO:0099637, neurotransmitter receptor localization to postsynaptic specialization membrane [GO:0099645], protein-containing complex localization to centriolar satellite [GO:0140706], Bub1-Bub3 complex localization to kinetochore [GO:1990299], intramanchette transport [GO:1990953] Relationships: is a type of macromolecule localization [GO:0033036] Sources: GOC:mah Also known as: establishment and maintenance of protein complex localization, protein complex localisation, cellular protein complex localisation, cellular protein complex localization, cellular protein-containing complex localization, establishment and maintenance of cellular protein complex localization, protein complex localization Definition: A localization process that acts on a protein complex; the complex is transported to, or maintained in, a specific location.